{
  "term_label": "regulation of signal transduction",
  "gene": "UniProtKB:P32298",
  "gene_name": "G protein-coupled receptor kinase 4",
  "term_id": "GO:0009966",
  "gene_symbol": "GRK4"
}